{
  "term_label": "plasma membrane",
  "term_id": "GO:0005886",
  "gene": "UniProtKB:Q5IJ48",
  "gene_symbol": "CRB2",
  "gene_name": "Protein crumbs homolog 2"
}